{
  "term_label": "beta-tubulin binding",
  "gene_symbol": "IFT74",
  "term_id": "GO:0048487",
  "gene": "UniProtKB:Q96LB3",
  "gene_name": "Intraflagellar transport protein 74 homolog"
}